{
  "gene_name": "Mannose-1-phosphate guanyltransferase alpha",
  "term_label": "Unknown biological process",
  "gene": "UniProtKB:Q96IJ6",
  "gene_symbol": "GMPPA",
  "term_id": "UNKNOWN:0002"
}